{
  "term_id": "GO:0005737",
  "gene": "UniProtKB:O00506",
  "gene_name": "Serine_threonine-protein kinase 25",
  "gene_symbol": "STK25",
  "term_label": "cytoplasm"
}